{
  "term_label": "extracellular matrix",
  "gene_name": "Metalloproteinase inhibitor 3",
  "gene": "UniProtKB:P35625",
  "term_id": "GO:0031012",
  "gene_symbol": "TIMP3"
}